{
  "term_id": "UNKNOWN:0001",
  "gene_symbol": "C3orf33",
  "gene_name": "Protein C3orf33",
  "term_label": "Unknown molecular function",
  "gene": "UniProtKB:Q6P1S2"
}